{
  "term_id": "GO:0061630",
  "term_label": "ubiquitin protein ligase activity",
  "gene": "UniProtKB:Q9C029",
  "gene_name": "E3 ubiquitin-protein ligase TRIM7",
  "gene_symbol": "TRIM7"
}